{
  "gene": "UniProtKB:Q9Y3B3",
  "term_label": "Golgi apparatus",
  "gene_symbol": "TMED7",
  "term_id": "GO:0005794",
  "gene_name": "Transmembrane emp24 domain-containing protein 7"
}